Oplophorus-luciferin 2-monooxygenase activity [GO:0033756] (molecular function) Sources: EC:1.13.12.13 Definition: Catalysis of the reaction: Oplophorus luciferin + O2 = oxidized Oplophorus luciferin + CO2 + hnu. Relationships: is a type of oxidoreductase activity, acting on single donors with incorporation of molecular oxygen, incorporation of one atom of oxygen (internal monooxygenases or internal mixed function oxidases) [GO:0016703]; is a type of luciferin monooxygenase activity [GO:0045289] Also known as: Oplophorus luciferase activity, Oplophorus-luciferin:oxygen 2-oxidoreductase (decarboxylating) activity